regulation of protein modification by small protein conjugation or removal [GO:1903320] (biological process) Definition: Any process that modulates the frequency, rate or extent of protein modification by small protein conjugation or removal. Sources: GOC:TermGenie, GOC:vw, GO_REF:0000058 Subtypes: GO:0031396, regulation of protein sumoylation [GO:0033233], GO:0060188, regulation of protein deneddylation [GO:0060625], regulation of protein deubiquitination [GO:0090085], negative regulation of protein modification by small protein conjugation or removal [GO:1903321], GO:1903322, GO:2000434 Relationships: is a type of regulation of post-translational protein modification [GO:1901873]; RO_0002211 protein modification by small protein conjugation or removal [GO:0070647]